{
  "gene": "UniProtKB:Q86U90",
  "gene_symbol": "YRDC",
  "gene_name": "Threonylcarbamoyl-AMP synthase",
  "term_label": "cytoplasm",
  "term_id": "GO:0005737"
}